negative regulation of neurotransmitter uptake [GO:0051581] (biological process) Definition: Any process that stops, prevents, or reduces the frequency, rate or extent of the directed movement of a neurotransmitter into a neuron or glial cell. Sources: GOC:ai Relationships: is a type of regulation of neurotransmitter uptake [GO:0051580]; is a type of GO:0051589; negatively regulates neurotransmitter uptake [GO:0001504] Subtypes: inhibition of neurotransmitter uptake [GO:0051609], negative regulation of serotonin uptake [GO:0051612], negative regulation of histamine uptake [GO:0051617], negative regulation of amino acid uptake involved in synaptic transmission [GO:0051942], negative regulation of catecholamine uptake involved in synaptic transmission [GO:0051945] Also known as: down regulation of neurotransmitter uptake, down-regulation of neurotransmitter uptake, downregulation of neurotransmitter uptake, negative regulation of neurotransmitter import